{
  "term_label": "nuclear speck",
  "gene_name": "Speckle targeted PIP5K1A-regulated poly(A) polymerase",
  "gene": "UniProtKB:Q9H6E5",
  "term_id": "GO:0016607",
  "gene_symbol": "TUT1"
}